neuronal-glial interaction involved in hindbrain glial-mediated radial cell migration [GO:0021944] (biological process) References: PMID:15157725 Sources: GOC:cls, GOC:dgh, GOC:dph, GOC:jid, GO_REF:0000021 Definition: The changes in adhesion between a neuronal cell and a glial cell as a component of the process of hindbrain glial-mediated radial cell migration. Relationships: is a type of cell-cell adhesion [GO:0098609]; is part of hindbrain radial glia guided cell migration [GO:0021932]